{
  "gene_name": "Single-pass membrane and coiled-coil domain-containing protein 3",
  "gene": "UniProtKB:A2RU48",
  "term_id": "UNKNOWN:0002",
  "gene_symbol": "SMCO3",
  "term_label": "Unknown biological process"
}